phosphatidylserine binding [GO:0001786] (molecular function) Relationships: is a type of phospholipid binding [GO:0005543]; is a type of anion binding [GO:0043168]; is a type of modified amino acid binding [GO:0072341] References: PMID:12000961 Sources: ISBN:0198506732 Definition: Binding to phosphatidylserine, a class of glycophospholipids in which a phosphatidyl group is esterified to the hydroxyl group of L-serine.